mitotic spindle elongation [GO:0000022] (biological process) Definition: The cell cycle process in which the distance is lengthened between poles of the mitotic spindle. Mitotic spindle elongation begins during mitotic prophase and ends during mitotic anaphase B. Relationships: is a type of spindle elongation [GO:0051231]; is_a mitotic cell cycle process [GO:1903047]; is part of GO:0000070; is part of GO:0007052 Regulation: regulated by GO:0032888; negatively regulated by negative regulation of mitotic spindle elongation [GO:1902845]; positively regulated by GO:1902846 Also known as: spindle elongation during mitosis, microtubule sliding involved in mitotic spindle elongation References: PMID:19686686 Sources: GOC:mtg_cell_cycle, GOC:vw